phosphatidylinositol transporter complex [GO:1902556] (cellular component) Definition: A protein complex which is capable of phosphatidylinositol transporter activity. References: PMID:9890948 Sources: GOC:TermGenie, GOC:bhm Note: An example is PDR16 in S. cerevisiae (UniProt ID P53860) in PMID:9890948 (inferred from direct assay). Relationships: is a type of transporter complex [GO:1990351]